{
  "gene_name": "Myeloid differentiation primary response protein MyD88",
  "term_id": "GO:0005886",
  "term_label": "plasma membrane",
  "gene": "UniProtKB:Q99836",
  "gene_symbol": "MYD88"
}